positive regulation of immunological synapse formation [GO:2000522] (biological process) Sources: GOC:obol Definition: Any process that activates or increases the frequency, rate or extent of immunological synapse formation. Also known as: positive regulation of formation of immunological synapse Relationships: is a type of GO:0048522; is a type of regulation of immunological synapse formation [GO:2000520]; positively regulates immunological synapse formation [GO:0001771]